{
  "gene_name": "Protein kinase C eta type",
  "term_label": "protein serine/threonine kinase activity",
  "term_id": "GO:0004674",
  "gene_symbol": "PRKCH",
  "gene": "UniProtKB:P24723"
}